protein retention in ER lumen [GO:0006621] (biological process) Definition: The retention in the endoplasmic reticulum (ER) lumen of soluble resident proteins. Sorting receptors retrieve proteins with ER localization signals, such as KDEL and HDEL sequences or some transmembrane domains, that have escaped to the cis-Golgi network and return them to the ER. Abnormally folded proteins and unassembled subunits are also selectively retained in the ER. Also known as: maintenance of protein location in ER lumen Relationships: is a type of maintenance of protein localization in endoplasmic reticulum [GO:0035437] References: PMID:12972550 Sources: ISBN:0716731363